{
  "term_label": "gamma-tubulin complex",
  "gene_name": "Gamma-tubulin complex component 2",
  "term_id": "GO:0000930",
  "gene": "UniProtKB:Q9BSJ2",
  "gene_symbol": "TUBGCP2"
}